{
  "gene_symbol": "PIP5KL1",
  "gene_name": "Phosphatidylinositol 4-phosphate 5-kinase-like protein 1",
  "term_label": "phosphatidylinositol phosphate biosynthetic process",
  "term_id": "GO:0046854",
  "gene": "UniProtKB:Q5T9C9"
}